{
  "gene_symbol": "ZEB2",
  "gene": "UniProtKB:O60315",
  "term_id": "GO:0000981",
  "term_label": "DNA-binding transcription factor activity, RNA polymerase II-specific",
  "gene_name": "Zinc finger E-box-binding homeobox 2"
}